{
  "term_label": "blood microparticle",
  "gene": "UniProtKB:P00736",
  "term_id": "GO:0072562",
  "gene_name": "Complement C1r subcomponent",
  "gene_symbol": "C1R"
}